tyramine-beta hydroxylase activity [GO:0004836] (molecular function) Definition: Catalysis of the reaction: tyramine + L-ascorbate + O2 = (R)-octopamine + L-dehydroascorbate + H2O. Relationships: is a type of oxidoreductase activity, acting on paired donors, with incorporation or reduction of molecular oxygen, reduced ascorbate as one donor, and incorporation of one atom of oxygen [GO:0016715] References: PMID:10745161 Sources: RHEA:57132